{
  "term_label": "positive regulation of transcription by RNA polymerase II",
  "gene": "UniProtKB:Q86YW9",
  "term_id": "GO:0045944",
  "gene_name": "Mediator of RNA polymerase II transcription subunit 12-like protein",
  "gene_symbol": "MED12L"
}